NK T cell activation involved in immune response [GO:0002288] (biological process) Relationships: is a type of GO:0002287; is a type of NK T cell activation [GO:0051132] Subtypes: NK T cell proliferation involved in immune response [GO:0002289] References: PMID:15771592 Sources: GOC:add Also known as: NK T cell activation during immune response, NK T lymphocyte activation during immune response, NK T-cell activation during immune response, NK T-lymphocyte activation during immune response, natural killer T lymphocyte activation during immune response, natural killer T-cell activation during immune response, natural killer T-lymphocyte activation during immune response Definition: The change in morphology and behavior of a mature or immature natural killer T cell resulting from exposure to a mitogen, cytokine, chemokine, cellular ligand, or an antigen for which it is specific, leading to the initiation or perpetuation of an immune response.